extracellular matrix constituent, lubricant activity [GO:0030197] (molecular function) Relationships: is a type of GO:0005201 Note: Extracellular matrix mucin proteins may be annotated to this term. PMID:14711375, PMID:18601586 Also known as: core extracellular matrix, core matrisome Definition: Functions as a lubricant for an extracellular matrix, such as a mucous membrane. Sources: GOC:mah